{
  "term_id": "UNKNOWN:0001",
  "term_label": "Unknown molecular function",
  "gene_symbol": "LNP1",
  "gene": "UniProtKB:A1A4G5",
  "gene_name": "Leukemia NUP98 fusion partner 1"
}